{
  "gene_symbol": "DUX4",
  "term_label": "regulation of transcription by RNA polymerase II",
  "gene_name": "Double homeobox protein 4",
  "term_id": "GO:0006357",
  "gene": "UniProtKB:Q9UBX2"
}